{
  "term_id": "GO:0006954",
  "gene_symbol": "TLR6",
  "term_label": "inflammatory response",
  "gene": "UniProtKB:Q9Y2C9",
  "gene_name": "Toll-like receptor 6"
}